{
  "term_label": "Rb-E2F complex",
  "gene_symbol": "E2F1",
  "term_id": "GO:0035189",
  "gene": "UniProtKB:Q01094",
  "gene_name": "Transcription factor E2F1"
}